{
  "term_id": "GO:0004674",
  "gene": "UniProtKB:Q96BR1",
  "term_label": "protein serine/threonine kinase activity",
  "gene_symbol": "SGK3",
  "gene_name": "Serine_threonine-protein kinase Sgk3"
}